{
  "gene": "UniProtKB:Q9BWU1",
  "term_label": "CKM complex",
  "gene_symbol": "CDK19",
  "term_id": "GO:1990508",
  "gene_name": "Cyclin-dependent kinase 19"
}